{
  "gene_name": "2'-5'-oligoadenylate synthase 2",
  "term_id": "GO:0003725",
  "gene": "UniProtKB:P29728",
  "gene_symbol": "OAS2",
  "term_label": "double-stranded RNA binding"
}